regulation of vascular associated smooth muscle cell apoptotic process [GO:1905459] (biological process) Definition: Any process that modulates the frequency, rate or extent of vascular associated smooth muscle cell apoptotic process. References: PMID:26493107 Sources: GOC:BHF, GOC:BHF_miRNA, GOC:TermGenie, GOC:rph, GO_REF:0000058 Also known as: regulation of VSMC apoptotic process, regulation of vascular smooth muscle cell apoptotic process, regulation of VSMC apoptosis, regulation of vascular associated smooth muscle cell apoptosis, regulation of vascular smooth muscle cell apoptosis Relationships: is a type of regulation of smooth muscle cell apoptotic process [GO:0034391]; regulates vascular associated smooth muscle cell apoptotic process [GO:1905288] Subtypes: GO:1905460, positive regulation of vascular associated smooth muscle cell apoptotic process [GO:1905461]